pinoresinol reductase activity [GO:0010283] (molecular function) Definition: Catalysis of the reaction: pinoresinol + NADPH + H+ = lariciresinol + NADP+. Relationships: is a type of oxidoreductase activity, reducing C-O-C group as acceptor [GO:0120546] References: PMID:10066819, PMID:7592828